{
  "term_label": "cytoplasmic vesicle",
  "gene": "UniProtKB:P84095",
  "gene_name": "Rho-related GTP-binding protein RhoG",
  "term_id": "GO:0031410",
  "gene_symbol": "RHOG"
}